{
  "term_id": "GO:0006357",
  "gene": "UniProtKB:O95343",
  "gene_symbol": "SIX3",
  "gene_name": "Homeobox protein SIX3",
  "term_label": "regulation of transcription by RNA polymerase II"
}